{
  "gene_symbol": "CBLL2",
  "term_id": "GO:0061630",
  "gene": "UniProtKB:Q8N7E2",
  "gene_name": "E3 ubiquitin-protein ligase CBLL2",
  "term_label": "ubiquitin protein ligase activity"
}